aldarate transmembrane transporter activity [GO:0042876] (molecular function) References: PMID:15034926 Sources: GOC:go_curators Subtypes: D-glucarate transmembrane transporter activity [GO:0042878], galactarate transmembrane transporter activity [GO:1902301] Definition: Enables the transfer of aldarate from one side of a membrane to the other. Relationships: is a type of carboxylic acid transmembrane transporter activity [GO:0046943]; is part of GO:0042869